{
  "gene_name": "Probable G-protein coupled receptor 34",
  "term_id": "GO:0045028",
  "gene": "UniProtKB:Q9UPC5",
  "term_label": "G protein-coupled purinergic nucleotide receptor activity",
  "gene_symbol": "GPR34"
}